{
  "term_id": "GO:0009986",
  "gene_symbol": "SDC4",
  "gene_name": "Syndecan-4",
  "gene": "UniProtKB:P31431",
  "term_label": "cell surface"
}